{
  "term_id": "GO:0017020",
  "gene_name": "Protein phosphatase 1 regulatory subunit 12C",
  "term_label": "myosin phosphatase regulator activity",
  "gene": "UniProtKB:Q9BZL4",
  "gene_symbol": "PPP1R12C"
}